{
  "term_id": "GO:2001234",
  "term_label": "negative regulation of apoptotic signaling pathway",
  "gene": "UniProtKB:P55061",
  "gene_name": "Bax inhibitor 1",
  "gene_symbol": "TMBIM6"
}